{
  "gene_symbol": "PPBP",
  "term_id": "GO:0030593",
  "gene": "UniProtKB:P02775",
  "gene_name": "Platelet basic protein",
  "term_label": "neutrophil chemotaxis"
}